{
  "term_id": "GO:0005737",
  "gene_name": "Sialidase-2",
  "term_label": "cytoplasm",
  "gene_symbol": "NEU2",
  "gene": "UniProtKB:Q9Y3R4"
}